{
  "gene": "UniProtKB:Q99719",
  "gene_symbol": "SEPTIN5",
  "gene_name": "Septin-5",
  "term_id": "GO:0031105",
  "term_label": "septin complex"
}